carbohydrate response element binding [GO:0035538] (molecular function) Relationships: is a type of GO:0000978 Definition: Binding to a carbohydrate response element (ChoRE) found in the promoters of genes whose expression is regulated in response to carbohydrates, such as the triglyceride synthesis genes. References: PMID:20001964 Sources: GOC:BHF Also known as: ChoRE binding